vitamin D 24-hydroxylase activity [GO:0070576] (molecular function) References: PMID:15546903 Sources: GOC:BHF, GOC:mah Definition: Catalysis of the hydroxylation of C-24 of any form of vitamin D. Also known as: calciferol 24-hydroxylase activity, cholecalciferol 24-hydroxylase activity, ergocalciferol 24-hydroxylase activity, vitamin D2 24-hydroxylase activity, vitamin D3 24-hydroxylase activity Relationships: is a type of steroid hydroxylase activity [GO:0008395] Subtypes: 25-hydroxycholecalciferol-24-hydroxylase activity [GO:0008403], 1-alpha,25-dihydroxyvitamin D3 24-hydroxylase activity [GO:0030342]